{
  "gene": "UniProtKB:Q96LU7",
  "term_id": "GO:0005789",
  "gene_name": "Myelin regulatory factor-like protein",
  "gene_symbol": "MYRFL",
  "term_label": "endoplasmic reticulum membrane"
}